{
  "term_id": "GO:0004842",
  "gene": "UniProtKB:Q5XPI4",
  "term_label": "ubiquitin-protein transferase activity",
  "gene_name": "E3 ubiquitin-protein ligase RNF123",
  "gene_symbol": "RNF123"
}